dihydroxyphenylalanine transaminase activity [GO:0047309] (molecular function) Also known as: dihydroxyphenylalanine aminotransferase activity, 3,4-dihydroxy-L-phenylalanine:2-oxoglutarate aminotransferase activity, DOPA aminotransferase activity, L-dopa transaminase activity, aspartate-DOPP transaminase (ADT), dopa transaminase activity, glutamate-DOPP transaminase (GDT), phenylalanine-DOPP transaminase (PDT) Sources: EC:2.6.1.49, RHEA:15273 Definition: Catalysis of the reaction: 2-oxoglutarate + L-dopa = 3,4-dihydroxyphenylpyruvate + L-glutamate. Relationships: is a type of transaminase activity [GO:0008483]